protein localization to actin filament bundle [GO:1903120] (BP) Definition: A process in which a protein is transported to, or maintained in, the location of an actin filament bundle. References: PMID:24798735 Sources: GOC:TermGenie, GO_REF:0000087 Also known as: protein localisation in actin filament bundle, protein localisation to actin filament bundle, protein localization in actin filament bundle, protein localization to actin cable Relationships: is a type of protein localization to actin cytoskeleton [GO:1903119]